{
  "gene_symbol": "HSP90AB1",
  "term_id": "GO:0034605",
  "gene_name": "Heat shock protein HSP 90-beta",
  "gene": "UniProtKB:P08238",
  "term_label": "cellular response to heat"
}